{
  "gene": "UniProtKB:P0DPK4",
  "gene_name": "Notch homolog 2 N-terminal-like protein C",
  "term_id": "GO:0005576",
  "gene_symbol": "NOTCH2NLC",
  "term_label": "extracellular region"
}